amorpha-4,11-diene 12-monooxygenase activity [GO:0062150] (molecular function) References: PMID:16458889, PMID:16612385, PMID:23246612 Sources: RHEA:32999 Definition: Catalysis of the reaction:(+)-amorpha-4,11-diene + 3 O2 + 3 reduced [NADPH--hemoprotein reductase] = (+)-artemisinate + 4 H+ + 4 H2O + 3 oxidized [NADPH--hemoprotein reductase]. Relationships: is a type of oxidoreductase activity, acting on paired donors, with incorporation or reduction of molecular oxygen [GO:0016705]